{
  "gene_symbol": "ZNF462",
  "gene_name": "Zinc finger protein 462",
  "term_id": "GO:0000976",
  "term_label": "transcription cis-regulatory region binding",
  "gene": "UniProtKB:Q96JM2"
}